{
  "gene_name": "Mdm2-binding protein",
  "gene_symbol": "MTBP",
  "gene": "UniProtKB:Q96DY7",
  "term_label": "kinetochore",
  "term_id": "GO:0000776"
}